{
  "gene_name": "T-complex protein 1 subunit beta",
  "gene_symbol": "CCT2",
  "term_label": "chaperonin-containing T-complex",
  "gene": "UniProtKB:P78371",
  "term_id": "GO:0005832"
}